cellular response to diethyl maleate [GO:1902112] (biological process) References: PMID:12100563 Sources: GOC:TermGenie Definition: Any process that results in a change in state or activity of a cell (in terms of movement, secretion, enzyme production, gene expression, etc.) as a result of a diethyl maleate stimulus. Relationships: is a type of cellular response to oxygen-containing compound [GO:1901701]; is a type of GO:1902111